{
  "term_label": "Unknown cellular component",
  "gene_name": "HCG2039775 (Fragment)",
  "gene_symbol": "TRAJ14",
  "term_id": "UNKNOWN:0003",
  "gene": "UniProtKB:A0N4Z3"
}